regulation of neutrophil aggregation [GO:2000428] (biological process) Definition: Any process that modulates the frequency, rate or extent of neutrophil aggregation. Sources: GOC:BHF Subtypes: GO:2000429, positive regulation of neutrophil aggregation [GO:2000430] Also known as: regulation of neutrocyte aggregation, regulation of neutrophil leucocyte aggregation, regulation of neutrophilic leukocyte aggregation Relationships: is a type of GO:1903037; regulates neutrophil aggregation [GO:0070488]